photosystem [GO:0009521] (cellular component) Relationships: is a type of membrane protein complex [GO:0098796]; is part of GO:0034357 Also known as: reaction center, reaction centre Definition: A complex located in a photosynthetic membrane that consists of a photoreaction center associated with accessory pigments and electron carriers. Examples of this component are found in Arabidopsis thaliana and in photosynthetic bacterial and archaeal species. References: PMID:9821949 Sources: GOC:ds, GOC:mah, ISBN:0140514031 Subtypes: photosystem I [GO:0009522], photosystem II [GO:0009523]